{
  "term_label": "cytoplasm",
  "gene_symbol": "PRAMEF15",
  "gene": "UniProtKB:P0DUQ1",
  "gene_name": "PRAME family member 15",
  "term_id": "GO:0005737"
}